taurine-pyruvate aminotransferase activity [GO:0031299] (molecular function) Relationships: is a type of transaminase activity [GO:0008483] References: PMID:11082195 Sources: RHEA:10420 Also known as: Tpa, taurine:pyruvate aminotransferase activity Definition: Catalysis of the reaction: pyruvate + taurine = L-alanine + sulfoacetaldehyde.